{
  "term_label": "virion binding",
  "gene_name": "Sialoadhesin",
  "gene": "UniProtKB:Q9BZZ2",
  "term_id": "GO:0046790",
  "gene_symbol": "SIGLEC1"
}